{
  "term_id": "GO:0048705",
  "gene_symbol": "COL11A2",
  "term_label": "skeletal system morphogenesis",
  "gene": "UniProtKB:P13942",
  "gene_name": "Collagen alpha-2(XI) chain"
}